{
  "gene_name": "Zinc finger protein 256",
  "term_label": "DNA-binding transcription factor activity, RNA polymerase II-specific",
  "gene_symbol": "ZNF256",
  "gene": "UniProtKB:Q9Y2P7",
  "term_id": "GO:0000981"
}